negative regulation of protein transport [GO:0051224] (biological process) Sources: GOC:ai Relationships: is a type of negative regulation of transport [GO:0051051]; is a type of GO:0051223; is a type of negative regulation of protein localization [GO:1903828]; is a type of negative regulation of establishment of protein localization [GO:1904950]; negatively regulates protein transport [GO:0015031] Also known as: down regulation of protein transport, down-regulation of protein transport, downregulation of protein transport, inhibition of protein transport Definition: Any process that stops, prevents, or reduces the frequency, rate or extent of the directed movement of a protein into, out of or within a cell, or between cells, by means of some agent such as a transporter or pore. Subtypes: negative regulation of Golgi to plasma membrane protein transport [GO:0042997], GO:0050709, negative regulation of intracellular protein transport [GO:0090317], GO:0140076, negative regulation of protein import [GO:1904590], negative regulation of ubiquitin-dependent endocytosis [GO:2000396]